{
  "gene_name": "Wilms tumor protein 1-interacting protein",
  "gene_symbol": "WTIP",
  "term_id": "GO:0003714",
  "gene": "UniProtKB:A6NIX2",
  "term_label": "transcription corepressor activity"
}